positive regulation of iron-sulfur cluster assembly [GO:1903331] (biological process) Definition: Any process that activates or increases the frequency, rate or extent of iron-sulfur cluster assembly. Also known as: positive regulation of iron-sulphur cluster assembly, up regulation of iron-sulfur cluster assembly, up regulation of iron-sulphur cluster assembly, up-regulation of iron-sulfur cluster assembly, up-regulation of iron-sulphur cluster assembly, upregulation of iron-sulfur cluster assembly, upregulation of iron-sulphur cluster assembly, activation of iron-sulfur cluster assembly, activation of iron-sulphur cluster assembly, activation of iron-sulfur cluster biosynthesis, positive regulation of iron-sulfur cluster biosynthesis, up regulation of iron-sulfur cluster biosynthesis, up-regulation of iron-sulfur cluster biosynthesis, upregulation of iron-sulfur cluster biosynthesis Sources: GOC:TermGenie, GOC:vw, GO_REF:0000058 Subtypes: positive regulation of [2Fe-2S] cluster assembly [GO:1900489], positive regulation of [4Fe-4S] cluster assembly [GO:1900493], positive regulation of iron-sulfur-molybdenum cofactor assembly [GO:1900508] Relationships: is a type of positive regulation of cellular component organization [GO:0051130]; is_a regulation of iron-sulfur cluster assembly [GO:1903329]; positively regulates GO:0016226